microtubule organizing center organization [GO:0031023] (biological process) Definition: A process that is carried out at the cellular level which results in the assembly, arrangement of constituent parts, or disassembly of a microtubule organizing center, a structure from which microtubules grow. Relationships: is a type of microtubule-based process [GO:0007017]; is a type of cellular component organization [GO:0016043]; is part of microtubule cytoskeleton organization [GO:0000226] Also known as: microtubule organising center organisation, microtubule organizing center organization and biogenesis Sources: GOC:dph, GOC:jl, GOC:mah Subtypes: GO:0007098, interphase microtubule organizing center assembly [GO:0031024], equatorial microtubule organizing center disassembly [GO:0031025], GO:0032053, spindle pole body organization [GO:0051300], centriole assembly [GO:0098534], equatorial microtubule organizing center assembly [GO:1904185]